D-leucine catabolic process [GO:1900832] (biological process) References: PMID:10918062 Sources: GOC:TermGenie Also known as: D-leucine breakdown, D-leucine catabolism, D-leucine degradation Relationships: is a type of branched-chain amino acid catabolic process [GO:0009083]; is a type of GO:0019478 Definition: The chemical reactions and pathways resulting in the breakdown of D-leucine.